{
  "gene_symbol": "CPHXL2",
  "term_label": "nucleus",
  "gene_name": "Cytoplasmic polyadenylated homeobox-like protein 2",
  "term_id": "GO:0005634",
  "gene": "UniProtKB:A0A1W2PPK0"
}